lactate:proton symporter activity [GO:0015650] (molecular function) Also known as: lactate permease, lactate:hydrogen porter activity, lactate:hydrogen symporter activity, lactate:proton porter activity Definition: Enables the transfer of a solute or solutes from one side of a membrane to the other according to the reaction: lactate (out) + H+ (out) = lactate (in) + H+ (in). Sources: TC:2.A.14.1.1 Relationships: is a type of lactate transmembrane transporter activity [GO:0015129]; is a type of GO:0015295; is a type of secondary active monocarboxylate transmembrane transporter activity [GO:0015355]